tryptophan sensor activity [GO:0120286] (MF) Definition: Binding to and responding, e.g. by conformational change, to changes in the cellular level of tryptophan. Also known as: tryptophan sensing activity Relationships: is a type of GO:0140785; has part GO:0120284 References: PMID:31498992 Sources: GOC:krc